fatty acid omega-1 hydroxylase activity [GO:0120502] (molecular function) Relationships: is a type of oxidoreductase activity, acting on paired donors, with incorporation or reduction of molecular oxygen, reduced flavin or flavoprotein as one donor, and incorporation of one atom of oxygen [GO:0016712] Sources: RHEA:44548 Definition: Catalysis of the reaction: an (omega-1)-ethyl fatty acid + O2 + reduced [NADPH--hemoprotein reductase] = an (omega-1)-hydroxy fatty acid + H+ + H2O + oxidized [NADPH--hemoprotein reductase]. Subtypes: long-chain fatty acid omega-1 hydroxylase activity [GO:0120319], medium-chain fatty acid omega-1 hydroxylase activity [GO:0120503]